immunoglobulin transcytosis in epithelial cells mediated by polymeric immunoglobulin receptor [GO:0002415] (biological process) Also known as: antibody transcytosis mediated by pIgR, immunoglobulin transcytosis mediated by pIgR Relationships: is a type of immunoglobulin transcytosis in epithelial cells [GO:0002414]; is part of mucosal immune response [GO:0002385] References: PMID:16048543 Sources: GOC:add, ISBN:0781735149, ISBN:081533642X Definition: The process of transporting polymeric IgA and polymeric IgM immunoglobulin, via transcytosis mediated by the polymeric immunoglobulin receptor (pIgR), from the basolateral surface to apical surface of an epithelial cell. At the apical surface the immunoglobulin binding portion of the pIgRis cleaved and remains bound to the transported immunoglobulin as secretory component (SC). The same process is used for the transport and excretion of IgA immune complexes to the luminal surface of the mucosa.